{
  "term_label": "calcineurin complex",
  "term_id": "GO:0005955",
  "gene": "UniProtKB:P16298",
  "gene_name": "Serine_threonine-protein phosphatase 2B catalytic subunit beta isoform",
  "gene_symbol": "PPP3CB"
}